{
  "term_label": "gastrin receptor activity",
  "gene": "UniProtKB:P32239",
  "gene_name": "Gastrin_cholecystokinin type B receptor",
  "gene_symbol": "CCKBR",
  "term_id": "GO:0015054"
}